{
  "term_id": "UNKNOWN:0003",
  "gene_symbol": "ANKRD20A12P",
  "gene_name": "Putative ankyrin repeat domain-containing protein 20A12 pseudogene",
  "term_label": "Unknown cellular component",
  "gene": "UniProtKB:Q8NF67"
}